{
  "gene": "UniProtKB:O75461",
  "term_id": "GO:0000981",
  "gene_symbol": "E2F6",
  "gene_name": "Transcription factor E2F6",
  "term_label": "DNA-binding transcription factor activity, RNA polymerase II-specific"
}